protein targeting to lysosome involved in chaperone-mediated autophagy [GO:0061740] (BP) Definition: The targeting of a protein to the lysosome process in which an input protein binds to a chaperone and subsequently to a lysosomal receptor. Relationships: is a type of protein targeting to lysosome [GO:0006622]; is_a protein targeting to vacuole involved in autophagy [GO:0071211]; is part of chaperone-mediated autophagy [GO:0061684]; has part signaling receptor binding [GO:0005102]; has part GO:0051087 References: PMID:22748206 Sources: GOC:PARL, GOC:dph, GOC:pad